pectic galactan metabolic process [GO:0010401] (BP) Sources: GOC:tair_curators Also known as: pectic galactan metabolism Relationships: is a type of rhamnogalacturonan I side chain metabolic process [GO:0010400] Definition: The chemical reactions and pathways involving galactan, a polymer of D-galactosyl units that can be found as a side chain of the pectin rhamnogalacturonan I.